{
  "gene_name": "tRNA (guanine(37)-N1)-methyltransferase",
  "gene_symbol": "TRMT5",
  "gene": "UniProtKB:Q32P41",
  "term_id": "GO:0070901",
  "term_label": "mitochondrial tRNA methylation"
}